{
  "term_label": "G protein-coupled receptor signaling pathway",
  "term_id": "GO:0007186",
  "gene_name": "P2Y purinoceptor 14",
  "gene_symbol": "P2RY14",
  "gene": "UniProtKB:Q15391"
}